galactolipase activity [GO:0047714] (molecular function) Also known as: 1,2-diacyl-3-beta-D-galactosyl-sn-glycerol acylhydrolase activity, galactolipid acylhydrolase activity, galactolipid lipase activity, polygalactolipase activity Relationships: is_a lipase activity [GO:0016298]; is_a GO:0052689 Sources: RHEA:13189 Definition: Catalysis of the reaction: a 1,2-diacyl-3-O-(beta-D-galactosyl)-sn-glycerol + 2 H2O = 3-beta-D-galactosyl-sn-glycerol + 2 a fatty acid + 2 H+.